{
  "term_id": "GO:0000978",
  "gene_name": "Hepatocyte nuclear factor 4-alpha",
  "gene": "UniProtKB:P41235",
  "term_label": "RNA polymerase II cis-regulatory region sequence-specific DNA binding",
  "gene_symbol": "HNF4A"
}